symbiont-mediated perturbation of host salicylic acid-mediated signal transduction pathway [GO:0052081] (BP) Also known as: modulation by organism of defense-related salicylic acid-mediated signal transduction pathway in other organism involved in symbiotic interaction, modulation by symbiont of defense-related host salicylic acid-mediated signal transduction pathway, modulation of defense-related host SA-mediated signal transduction pathway by organism, perturbation of defense-related host salicylic acid-mediated signal transduction pathway Subtypes: symbiont-mediated suppression of defense-related host salicylic acid-mediated signal transduction pathway [GO:0052003] References: PMID:35698792 Sources: GOC:mtg_pamgo_17jul06 Relationships: is a type of symbiont-mediated perturbation of host signal transduction pathway [GO:0052027] Definition: A process in which a symbiont alters or subverts a salicylic acid-mediated signal transduction pathway in its host. The host is defined as the larger of the organisms involved in a symbiotic interaction.